cellular response to mycophenolic acid [GO:0071506] (biological process) Also known as: cellular response to mycophenolate Definition: Any process that results in a change in state or activity of a cell (in terms of movement, secretion, enzyme production, gene expression, etc.) as a result of a mycophenolic acid stimulus. Sources: GOC:mah, GOC:yaf Relationships: is a type of response to mycophenolic acid [GO:0071505]; is a type of cellular response to oxygen-containing compound [GO:1901701]